{
  "term_label": "6-phosphofructokinase activity",
  "gene_symbol": "PFKL",
  "gene_name": "ATP-dependent 6-phosphofructokinase, liver type",
  "gene": "UniProtKB:P17858",
  "term_id": "GO:0003872"
}